myeloid cell homeostasis [GO:0002262] (biological process) Sources: CL:0000763, GOC:add Definition: The process of regulating the proliferation and elimination of myeloid cells such that the total number of myeloid cells within a whole or part of an organism is stable over time in the absence of an outside stimulus. Subtypes: neutrophil homeostasis [GO:0001780], mast cell homeostasis [GO:0033023], GO:0034101, monocyte homeostasis [GO:0035702], macrophage homeostasis [GO:0061519], eosinophil homeostasis [GO:1990959], basophil homeostasis [GO:1990960] Relationships: is a type of GO:0002376; is a type of homeostasis of number of cells [GO:0048872]